hydrolase activity, hydrolyzing O-glycosyl compounds [GO:0004553] (molecular function) Also known as: O-glucosyl hydrolase activity Definition: Catalysis of the hydrolysis of any O-glycosyl bond. Relationships: is a type of hydrolase activity, acting on glycosyl bonds [GO:0016798] Subtypes: GO:0000016, lysozyme activity [GO:0003796], GO:0003940, GO:0004564, chitinase activity [GO:0004568], poly(ADP-ribose) glycohydrolase activity [GO:0004649], GO:0004650, cellulase activity [GO:0008810], limit dextrinase activity [GO:0010303], mannosidase activity [GO:0015923], GO:0015925, GO:0015926, GO:0015927, fucosidase activity [GO:0015928], hexosaminidase activity [GO:0015929], amylase activity [GO:0016160], cellulose 1,4-beta-cellobiosidase activity [GO:0016162], GO:0016977, alpha-sialidase activity [GO:0016997], glycosylceramidase activity [GO:0017042], GO:0019137, isoamylase activity [GO:0019156], GO:0030305, GO:0030596, GO:0031216, levanase activity [GO:0031219], dextranase activity [GO:0033904], GO:0033908, fucoidanase activity [GO:0033909], glucan 1,4-alpha-maltotetraohydrolase activity [GO:0033910], GO:0033911, 2,6-beta-fructan 6-levanbiohydrolase activity [GO:0033912], beta-agarase activity [GO:0033916], exo-poly-alpha-galacturonosidase activity [GO:0033917], kappa-carrageenase activity [GO:0033918], peptidoglycan beta-N-acetylmuramidase activity [GO:0033922], glucan 1,6-alpha-isomaltosidase activity [GO:0033923], dextran 1,6-alpha-isomaltotriosidase activity [GO:0033924], mannosyl-glycoprotein endo-beta-N-acetylglucosaminidase activity [GO:0033925], GO:0033926, glucan 1,4-alpha-maltohexaosidase activity [GO:0033927], GO:0033928, GO:0033934, GO:0033936, 3-deoxy-2-octulosonidase activity [GO:0033937], GO:0033939, 4-alpha-D-(1->4)-alpha-D-glucanotrehalose trehalohydrolase activity [GO:0033942], beta-galactofuranosidase activity [GO:0033944], oligoxyloglucan reducing-end-specific cellobiohydrolase activity [GO:0033945], fructan beta-(2,1)-fructosidase activity [GO:0033948], fructan beta-(2,6)-fructosidase activity [GO:0033949], oligosaccharide reducing-end xylanase activity [GO:0033951], iota-carrageenase activity [GO:0033952], alpha-agarase activity [GO:0033953], GO:0033954, lambda-carrageenase activity [GO:0033957], GO:0042972, glucan 1,4-alpha-maltohydrolase activity [GO:0043897], alpha-L-arabinofuranosidase activity [GO:0046556], arabinan endo-1,5-alpha-L-arabinosidase activity [GO:0046558], glucuronidase activity [GO:0046574], lacto-N-biosidase activity [GO:0047403], beta-L-arabinosidase activity [GO:0047701], cyclomaltodextrinase activity [GO:0047798], difructose-anhydride synthase activity [GO:0047853], endoglycosylceramidase activity [GO:0047876], GO:0047911, 3-deoxyoctulosonase activity [GO:0050534], beta-primeverosidase activity [GO:0050535], GO:0051060, GO:0051669, inulinase activity [GO:0051670], GO:0051675, beta-glucanase activity [GO:0052736], exo-1,4-beta-D-glucosaminidase activity [GO:0052761], beta-6-sulfate-N-acetylglucosaminidase activity [GO:0052769], endo-1,3-alpha-L-rhamnosidase activity [GO:0052775], d-4,5 unsaturated beta-glucuronyl hydrolase activity [GO:0052788], endo-xylogalacturonan hydrolase activity [GO:0052792], alpha-D-xyloside xylohydrolase [GO:0061634], xyloglucan 1,6-alpha-xylosidase activity [GO:0080176], xylanase activity [GO:0097599], GO:0102211, GO:0102212, GO:0102224, cellulose 1,4-beta-cellobiosidase activity (reducing end) [GO:0102252], 2-acetamido-4-O-(2-amino-2-deoxy-beta-D-glucopyranosyl)-2-deoxy-D-glucose exo-beta-D-glucosaminidase activity [GO:0102277], UDP-N,N'-diacetylbacillosamine 2-epimerase activity [GO:0102388], 6-O-methyl-deacetylisoipecoside beta-glucosidase activity [GO:0102413], beta-L-arabinofuranosidase activity [GO:0102478], [protein]-3-O-(N-acetyl-D-glucosaminyl)-L-serine/L-threonine O-N-acetyl-alpha-D-glucosaminase activity [GO:0102571], GO:0102726, dalcochinase activity [GO:0102954], GO:0120549, phlorizin hydrolase activity [GO:0140749] Sources: GOC:mah